{
  "gene_name": "Tetratricopeptide repeat protein 39A",
  "gene_symbol": "TTC39A",
  "gene": "UniProtKB:Q5SRH9",
  "term_id": "UNKNOWN:0001",
  "term_label": "Unknown molecular function"
}